pentalenolactone catabolic process [GO:1901779] (biological process) Definition: The chemical reactions and pathways resulting in the breakdown of pentalenolactone. References: PMID:17178094 Sources: GOC:TermGenie, GOC:yaf Also known as: pentalenolactone breakdown, pentalenolactone catabolism, pentalenolactone degradation Relationships: is a type of sesquiterpenoid catabolic process [GO:0016107]; is a type of monocarboxylic acid catabolic process [GO:0072329]; is a type of epoxide metabolic process [GO:0097176]; is a type of lactone catabolic process [GO:1901335]; is a type of ether catabolic process [GO:1901502]